{
  "gene_symbol": "EHD4",
  "gene": "UniProtKB:Q9H223",
  "term_id": "GO:0060271",
  "term_label": "cilium assembly",
  "gene_name": "EH domain-containing protein 4"
}